{
  "gene_name": "Immunoglobulin subtype domain-containing protein",
  "gene": "UniProtKB:A0A5F9ZH88",
  "term_label": "immune receptor activity",
  "term_id": "GO:0140375",
  "gene_symbol": "A0A5F9ZH88"
}